{
  "term_label": "mitochondrion",
  "gene": "UniProtKB:P52790",
  "gene_name": "Hexokinase-3",
  "term_id": "GO:0005739",
  "gene_symbol": "HK3"
}